{
  "gene": "UniProtKB:Q7Z6J8",
  "term_id": "GO:0006513",
  "gene_symbol": "UBE3D",
  "gene_name": "E3 ubiquitin-protein ligase E3D",
  "term_label": "protein monoubiquitination"
}